{
  "term_label": "protein quality control for misfolded or incompletely synthesized proteins",
  "gene_name": "Metalloendopeptidase OMA1, mitochondrial",
  "gene": "UniProtKB:Q96E52",
  "gene_symbol": "OMA1",
  "term_id": "GO:0006515"
}